nitrate efflux transmembrane transporter activity [GO:0010542] (MF) Relationships: is_a GO:0015513; is a type of efflux transmembrane transporter activity [GO:0015562] Definition: Enables the transfer of nitrate from the inside of the cell to the outside of the cell across a membrane. Sources: GOC:mah